detection of bacterial lipoprotein [GO:0042494] (biological process) Definition: The series of events in which a bacterial lipoprotein stimulus is received by a cell and converted into a molecular signal. Bacterial lipoproteins are lipoproteins characterized by the presence of conserved sequence motifs called pathogen-associated molecular patterns (PAMPs). References: PMID:12077222 Sources: GOC:jl Also known as: detection of BLP, detection of Lpp, perception of BLP, perception of Lpp, perception of bacterial lipoprotein Relationships: is a type of detection of molecule of bacterial origin [GO:0032490]; is a type of response to bacterial lipoprotein [GO:0032493]; is part of GO:0016045 Subtypes: GO:0070340